{
  "gene_name": "Catenin alpha-1",
  "term_id": "GO:0098609",
  "gene": "UniProtKB:P35221",
  "term_label": "cell-cell adhesion",
  "gene_symbol": "CTNNA1"
}